negative regulation of lateral motor column neuron migration [GO:1902077] (biological process) Also known as: down regulation of lateral motor column neuron migration, down-regulation of lateral motor column neuron migration, downregulation of lateral motor column neuron migration, inhibition of lateral motor column neuron migration Definition: Any process that stops, prevents or reduces the frequency, rate or extent of lateral motor column neuron migration. Relationships: is a type of regulation of lateral motor column neuron migration [GO:1902076]; is a type of negative regulation of motor neuron migration [GO:1905484]; negatively regulates lateral motor column neuron migration [GO:0097477] References: PMID:20711475 Sources: GOC:TermGenie, GOC:yaf